{
  "term_id": "GO:0005737",
  "term_label": "cytoplasm",
  "gene": "UniProtKB:Q92597",
  "gene_name": "Protein NDRG1",
  "gene_symbol": "NDRG1"
}